{
  "gene_name": "N-acetyltransferase 8",
  "gene_symbol": "NAT8",
  "term_label": "Unknown biological process",
  "term_id": "UNKNOWN:0002",
  "gene": "UniProtKB:Q9UHE5"
}